{
  "gene_name": "Small proline-rich protein 3",
  "term_id": "UNKNOWN:0002",
  "term_label": "Unknown biological process",
  "gene_symbol": "SPRR3",
  "gene": "UniProtKB:Q9UBC9"
}